{
  "term_id": "UNKNOWN:0003",
  "gene": "UniProtKB:Q9UPC5",
  "gene_symbol": "GPR34",
  "gene_name": "Probable G-protein coupled receptor 34",
  "term_label": "Unknown cellular component"
}